symbiont-mediated suppression of host synaptic transmission [GO:0044759] (biological process) Relationships: is a type of symbiont-mediated perturbation of host synaptic transmission [GO:0044758] Definition: A process in which a symbiont inhibits or disrupts the normal execution of synaptic transmission, communication from a neuron to a target (neuron, muscle, or secretory cell) across a synapse, in its host organism. Also known as: negative regulation by symbiont of host synaptic transmission Subtypes: symbiont-mediated suppression of host cholinergic synaptic transmission [GO:0044761] Sources: GOC:jl